{
  "gene_symbol": "UGT1A10",
  "gene": "UniProtKB:Q9HAW8",
  "term_id": "GO:0005783",
  "gene_name": "UDP-glucuronosyltransferase 1A10",
  "term_label": "endoplasmic reticulum"
}